positive regulation of sensory perception of sweet taste [GO:1904658] (biological process) Definition: Any process that activates or increases the frequency, rate or extent of sensory perception of sweet taste. Relationships: is_a positive regulation of nervous system process [GO:0031646]; is a type of regulation of sensory perception of sweet taste [GO:1904656]; positively regulates GO:0050916 References: PMID:1716172 Sources: GOC:TermGenie, GOC:mr, GO_REF:0000058 Also known as: positive regulation of sweet taste perception, up regulation of sensory perception of sweet taste, up regulation of sweet taste perception, up-regulation of sensory perception of sweet taste, up-regulation of sweet taste perception, upregulation of sensory perception of sweet taste, upregulation of sweet taste perception, activation of sensory perception of sweet taste, activation of sweet taste perception